{
  "term_label": "nucleus",
  "term_id": "GO:0005634",
  "gene_symbol": "YAF2",
  "gene_name": "YY1-associated factor 2",
  "gene": "UniProtKB:Q8IY57"
}